{
  "gene_symbol": "PACSIN3",
  "term_id": "GO:0030100",
  "term_label": "regulation of endocytosis",
  "gene_name": "Protein kinase C and casein kinase substrate in neurons protein 3",
  "gene": "UniProtKB:Q9UKS6"
}